{
  "term_id": "GO:0005634",
  "gene_symbol": "ZC3H14",
  "term_label": "nucleus",
  "gene": "UniProtKB:Q6PJT7",
  "gene_name": "Zinc finger CCCH domain-containing protein 14"
}